{
  "term_label": "chromatin binding",
  "gene_name": "Scm-like with four MBT domains protein 2",
  "gene_symbol": "SFMBT2",
  "gene": "UniProtKB:Q5VUG0",
  "term_id": "GO:0003682"
}